{
  "term_label": "Unknown molecular function",
  "gene_name": "Coenzyme Q-binding protein COQ10 homolog B, mitochondrial",
  "gene": "UniProtKB:Q9H8M1",
  "gene_symbol": "COQ10B",
  "term_id": "UNKNOWN:0001"
}